{
  "gene_name": "Cytosolic Fe-S cluster assembly factor NUBP1",
  "gene": "UniProtKB:P53384",
  "term_id": "GO:0005829",
  "gene_symbol": "NUBP1",
  "term_label": "cytosol"
}